{
  "gene_name": "Kinesin-like protein KIF26B",
  "gene_symbol": "KIF26B",
  "term_id": "GO:0008017",
  "gene": "UniProtKB:Q2KJY2",
  "term_label": "microtubule binding"
}